{
  "gene": "UniProtKB:P05154",
  "gene_name": "Plasma serine protease inhibitor",
  "term_id": "UNKNOWN:0002",
  "gene_symbol": "SERPINA5",
  "term_label": "Unknown biological process"
}